{
  "term_id": "UNKNOWN:0003",
  "term_label": "Unknown cellular component",
  "gene_symbol": "TSTD3",
  "gene": "UniProtKB:H0UI37",
  "gene_name": "Thiosulfate sulfurtransferase_rhodanese-like domain-containing protein 3"
}